{
  "gene": "UniProtKB:P18825",
  "gene_name": "Alpha-2C adrenergic receptor",
  "term_label": "plasma membrane",
  "term_id": "GO:0005886",
  "gene_symbol": "ADRA2C"
}